{
  "gene_symbol": "CFAP47",
  "gene": "UniProtKB:Q6ZTR5",
  "gene_name": "Cilia- and flagella-associated protein 47",
  "term_id": "GO:0007288",
  "term_label": "sperm axoneme assembly"
}